{
  "gene_symbol": "FAS",
  "term_id": "GO:0097527",
  "gene": "UniProtKB:P25445",
  "term_label": "necroptotic signaling pathway",
  "gene_name": "Tumor necrosis factor receptor superfamily member 6"
}